{
  "gene_symbol": "OTOL1",
  "term_id": "UNKNOWN:0001",
  "gene": "UniProtKB:A6NHN0",
  "gene_name": "Otolin-1",
  "term_label": "Unknown molecular function"
}